{
  "term_label": "Golgi apparatus",
  "gene": "UniProtKB:Q9NQX7",
  "term_id": "GO:0005794",
  "gene_name": "Integral membrane protein 2C",
  "gene_symbol": "ITM2C"
}